negative regulation of protein polyubiquitination [GO:1902915] (biological process) References: PMID:23645667 Sources: GOC:TermGenie, GOC:di, GO_REF:0000058 Subtypes: negative regulation of protein K48-linked ubiquitination [GO:0061944], negative regulation of protein K63-linked ubiquitination [GO:1900045], negative regulation of protein linear polyubiquitination [GO:1902529] Definition: Any process that stops, prevents or reduces the frequency, rate or extent of protein polyubiquitination. Relationships: is a type of GO:0031397; is a type of GO:1902914; negatively regulates protein polyubiquitination [GO:0000209] Also known as: down regulation of protein polyubiquitination, down regulation of protein polyubiquitinylation, down regulation of protein polyubiquitylation, down-regulation of protein polyubiquitination, down-regulation of protein polyubiquitinylation, down-regulation of protein polyubiquitylation, downregulation of protein polyubiquitination, downregulation of protein polyubiquitinylation, downregulation of protein polyubiquitylation, negative regulation of protein polyubiquitinylation, negative regulation of protein polyubiquitylation, inhibition of protein polyubiquitination, inhibition of protein polyubiquitinylation, inhibition of protein polyubiquitylation, down regulation of polyubiquitin, down-regulation of polyubiquitin, downregulation of polyubiquitin, inhibition of polyubiquitin, negative regulation of polyubiquitin